negative regulation of turning behavior involved in mating [GO:0061096] (biological process) Sources: GOC:dph, GOC:tb Relationships: is a type of regulation of turning behavior involved in mating [GO:0061094]; is a type of negative regulation of male mating behavior [GO:1902436]; negatively regulates turning behavior involved in mating [GO:0034607] Definition: Any process that decreases the rate, frequency or extent of turning behavior involved in mating. Turning behavior is the sharp ventral turn performed by the male as he approaches either the hermaphrodite head or tail, whilst trying to locate his partner's vulva. Turning occurs via a sharp ventral coil of the male's tail.